{
  "term_label": "proteolysis",
  "gene_name": "Pepsin A-5",
  "gene": "UniProtKB:P0DJD9",
  "term_id": "GO:0006508",
  "gene_symbol": "PGA5"
}